GATA1-TAL1-TCF3-Lmo2 complex [GO:0070353] (cellular component) Relationships: is a type of GO:0140513 Definition: A protein complex that contains the zinc finger transcription factor GATA1, the LIM domain protein Lmo2 (RBTN2), the basic helix-loop-helix protein TAL1 and its binding partner TCF3. The complex is involved transcriptional regulation in hematopoiesis. References: PMID:7568177